peptidoglycan immune receptor activity [GO:0016019] (molecular function) References: PMID:14698226 Note: Note that only peptidoglycan recognition proteins with receptor activity should be annotated to this term; otherwise use 'peptidoglycan binding ; GO:0042834' instead. Definition: Combining with a peptidoglycan and transmitting the signal to initiate an innate immune response. Relationships: is a type of pattern recognition receptor activity [GO:0038187]; has part peptidoglycan binding [GO:0042834] Also known as: peptidoglycan receptor activity, peptidoglycan recognition activity